glucosidase complex [GO:1902687] (cellular component) Subtypes: glucosidase II complex [GO:0017177], sucrase-isomaltase complex [GO:0070014] Definition: A protein complex which is capable of glucosidase activity. References: PMID:23826932 Sources: GOC:TermGenie, GOC:bhm, GO_REF:0000088 Note: An example of this is ygjK in E. coli (P42592) in PMID:23826932. Relationships: is a type of catalytic complex [GO:1902494]